dendritic tuft [GO:0044296] (cellular component) Sources: NIF_Subcellular:sao1340260079 Also known as: dendrite tuft Definition: The terminal specialization found in some types of dendrites which consists of numerous small terminal branches, giving the dendrite a tufted appearance. Relationships: is a type of dendrite terminus [GO:0044292]